positive regulation of plasma membrane bounded cell projection assembly [GO:0120034] (biological process) Definition: Any process that activates or increases the frequency, rate or extent of plasma membrane bounded cell projection assembly. Subtypes: positive regulation of lamellipodium assembly [GO:0010592], positive regulation of pseudopodium assembly [GO:0031274], positive regulation of cilium assembly [GO:0045724], GO:0051491, positive regulation of ruffle assembly [GO:1900029], positive regulation of mating projection assembly [GO:1902917], positive regulation of microvillus assembly [GO:1903698], positive regulation of bleb assembly [GO:1904172], positive regulation of dendritic cell dendrite assembly [GO:2000549] Sources: GOC:krc Relationships: is a type of positive regulation of cell projection organization [GO:0031346]; is a type of positive regulation of cellular component biogenesis [GO:0044089]; is a type of regulation of plasma membrane bounded cell projection assembly [GO:0120032]; positively regulates plasma membrane bounded cell projection assembly [GO:0120031]